{
  "gene": "UniProtKB:Q16763",
  "term_label": "protein polyubiquitination",
  "gene_symbol": "UBE2S",
  "term_id": "GO:0000209",
  "gene_name": "Ubiquitin-conjugating enzyme E2 S"
}